positive regulation of epinephrine uptake [GO:0051628] (biological process) Relationships: is a type of positive regulation of transport [GO:0051050]; is a type of GO:0051626; positively regulates epinephrine uptake [GO:0051625] Sources: GOC:ai Also known as: positive regulation of adrenaline uptake, positive regulation of epinephrine import, up regulation of epinephrine uptake, up-regulation of epinephrine uptake, upregulation of epinephrine uptake, activation of epinephrine uptake, stimulation of epinephrine uptake Definition: Any process that activates or increases the frequency, rate or extent of the directed movement of epinephrine into a cell.